AMP-activated protein kinase activity [GO:0004679] (molecular function) Sources: GOC:mah Relationships: is_a GO:0004674; has part AMP binding [GO:0016208] Definition: Catalysis of the reaction: ATP + a protein = ADP + a phosphoprotein. This reaction requires the presence of AMP. Also known as: 5'-AMP-activated protein kinase activity, protein kinase A activity, SNF1A/AMP-activated protein kinase activity, AMPK activity